polyprenyl diphosphate synthase complex [GO:0032476] (cellular component) Subtypes: homodimeric polyprenyl diphosphate synthase complex [GO:0032477], heterotetrameric polyprenyl diphosphate synthase complex [GO:0032478], dehydrodolichyl diphosphate synthase complex [GO:1904423] Also known as: decaprenyl diphosphate synthase complex Relationships: is_a GO:1990234 Definition: A complex that possesses polyprenyl diphosphate synthase activity involved in the synthesis of the isoprenoid chain of ubiquinone whose length varies between organisms. References: PMID:14519123, PMID:16262699 Sources: GOC:mah